L-methionine catabolic process [GO:0009087] (biological process) Relationships: is a type of sulfur amino acid catabolic process [GO:0000098]; is a type of methionine metabolic process [GO:0006555]; is_a L-amino acid catabolic process [GO:0170035]; is a type of proteinogenic amino acid catabolic process [GO:0170040] Definition: The chemical reactions and pathways resulting in the breakdown of L-methionine (2-amino-4-(methylthio)butanoic acid), a sulfur-containing, essential amino acid found in peptide linkage in proteins. Also known as: methionine breakdown, methionine catabolism, methionine degradation Subtypes: GO:0000951, GO:0000954, L-methionine catabolic process to succinyl-CoA [GO:0019457], L-methionine catabolic process via 2-oxobutanoate [GO:0019458] Sources: GOC:jl, ISBN:0198506732